dicarboxylic acid biosynthetic process [GO:0043650] (biological process) Relationships: is a type of dicarboxylic acid metabolic process [GO:0043648]; is a type of GO:0046394 Definition: The chemical reactions and pathways resulting in the formation of dicarboxylic acids, any organic acid containing two carboxyl (-COOH) groups. Also known as: dicarboxylate biosynthesis, dicarboxylate biosynthetic process, dicarboxylic acid anabolism, dicarboxylic acid biosynthesis, dicarboxylic acid formation, dicarboxylic acid synthesis Subtypes: GO:0006532, glutamate biosynthetic process [GO:0006537], GO:0006761, 10-formyltetrahydrofolate biosynthetic process [GO:0009257], GO:0009423, phytochromobilin biosynthetic process [GO:0010024], L-tyrosine catabolic process to fumarate [GO:0019445], glutamate catabolic process to oxaloacetate [GO:0019554], GO:0019578, GO:0019805, diaminopimelate biosynthetic process [GO:0019877], gibberellin 12 biosynthetic process [GO:0033470], GO:0033610, Kdo2-lipid A biosynthetic process [GO:0036104], folic acid biosynthetic process [GO:0046656], actinorhodin biosynthetic process [GO:1901112], 5,6,7,8-tetrahydromethanopterin biosynthetic process [GO:1901285], prephenate(2-) biosynthetic process [GO:1901747] Sources: ISBN:0198506732